{
  "gene_symbol": "GOLGA6L6",
  "gene": "UniProtKB:A8MZA4",
  "term_label": "Unknown cellular component",
  "gene_name": "Golgin subfamily A member 6-like protein 6",
  "term_id": "UNKNOWN:0003"
}